{
  "term_id": "GO:0035965",
  "term_label": "cardiolipin acyl-chain remodeling",
  "gene_name": "85_88 kDa calcium-independent phospholipase A2",
  "gene": "UniProtKB:O60733",
  "gene_symbol": "PLA2G6"
}